{
  "gene_symbol": "ADCYAP1",
  "term_label": "neuropeptide hormone activity",
  "gene": "UniProtKB:P18509",
  "term_id": "GO:0005184",
  "gene_name": "Pituitary adenylate cyclase-activating polypeptide"
}